{
  "term_label": "Unknown cellular component",
  "gene": "UniProtKB:Q6ZRG5",
  "gene_symbol": "Q6ZRG5",
  "term_id": "UNKNOWN:0003",
  "gene_name": "Putative uncharacterized protein FLJ43944"
}